{
  "gene_symbol": "ERN2",
  "gene_name": "Serine_threonine-protein kinase_endoribonuclease IRE2",
  "term_id": "GO:0036498",
  "term_label": "IRE1-mediated unfolded protein response",
  "gene": "UniProtKB:Q76MJ5"
}